{
  "gene_name": "Ras-related protein R-Ras2",
  "gene": "UniProtKB:P62070",
  "gene_symbol": "RRAS2",
  "term_label": "plasma membrane",
  "term_id": "GO:0005886"
}